{
  "gene": "UniProtKB:Q5W5W9",
  "gene_symbol": "RESP18",
  "term_label": "endoplasmic reticulum",
  "gene_name": "Regulated endocrine-specific protein 18",
  "term_id": "GO:0005783"
}